phosphotyrosine residue binding [GO:0001784] (molecular function) Definition: Binding to a phosphorylated tyrosine residue within a protein. References: PMID:14636584 Also known as: phosphotyrosine binding Relationships: is a type of GO:0045309